{
  "gene": "UniProtKB:P29728",
  "term_id": "GO:0060337",
  "gene_name": "2'-5'-oligoadenylate synthase 2",
  "gene_symbol": "OAS2",
  "term_label": "type I interferon-mediated signaling pathway"
}